{
  "gene_symbol": "SPDYE13",
  "term_label": "Unknown cellular component",
  "gene_name": "Putative speedy protein E13",
  "gene": "UniProtKB:A0A494C0Z2",
  "term_id": "UNKNOWN:0003"
}